{
  "gene_symbol": "MEN1",
  "term_label": "histone methyltransferase complex",
  "gene": "UniProtKB:O00255",
  "term_id": "GO:0035097",
  "gene_name": "Menin"
}